{
  "gene": "UniProtKB:Q9NQC1",
  "term_label": "regulation of transcription by RNA polymerase II",
  "gene_name": "E3 ubiquitin-protein ligase Jade-2",
  "gene_symbol": "JADE2",
  "term_id": "GO:0006357"
}